{
  "term_id": "GO:0070492",
  "gene_symbol": "SELE",
  "term_label": "oligosaccharide binding",
  "gene": "UniProtKB:P16581",
  "gene_name": "E-selectin"
}